cyclization of glutamine involved in intein-mediated protein splicing [GO:0019802] (biological process) Also known as: cyclization of glutamine, during protein splicing Definition: The cyclization of glutamine to yield an L-glutamimide residue at the C-terminus of an excised intein during protein splicing. Relationships: is a type of glutamine metabolic process [GO:0006541]; is part of intein-mediated protein splicing [GO:0016539] Sources: GOC:dph, GOC:tb, RESID:AA0303 Note: Note that this term should not be confused with 'peptidyl-pyroglutamic acid biosynthesis, using glutaminyl-peptide cyclotransferase ; GO:0017186'. See also the biological process term 'intein-mediated protein splicing ; GO:0016539'.